{
  "gene": "UniProtKB:Q9UKV3",
  "term_label": "Unknown molecular function",
  "term_id": "UNKNOWN:0001",
  "gene_symbol": "ACIN1",
  "gene_name": "Apoptotic chromatin condensation inducer in the nucleus"
}